{
  "gene_name": "Sister chromatid cohesion protein PDS5 homolog B",
  "gene_symbol": "PDS5B",
  "term_id": "GO:0000785",
  "term_label": "chromatin",
  "gene": "UniProtKB:Q9NTI5"
}